{
  "gene_symbol": "FASLG",
  "term_label": "cytokine activity",
  "gene_name": "Tumor necrosis factor ligand superfamily member 6",
  "term_id": "GO:0005125",
  "gene": "UniProtKB:P48023"
}